nucleus [GO:0005634] (CC) Relationships: is a type of intracellular membrane-bounded organelle [GO:0043231] Also known as: cell nucleus, horsetail nucleus Definition: A membrane-bounded organelle of eukaryotic cells in which chromosomes are housed and replicated. In most cells, the nucleus contains all of the cell's chromosomes except the organellar chromosomes, and is the site of RNA synthesis and processing. In some species, or in specialized cell types, RNA metabolism or DNA replication may be absent. Sources: GOC:go_curators Subtypes: GO:0031039, micronucleus [GO:0031040], germ cell nucleus [GO:0043073], megasporocyte nucleus [GO:0043076], pronucleus [GO:0045120], primary endosperm nucleus [GO:0048353], generative cell nucleus [GO:0048555], microsporocyte nucleus [GO:0048556], left nucleus [GO:0097571], right nucleus [GO:0097572], ascospore-type prospore nucleus [GO:1905754]